{
  "term_label": "cytoplasm",
  "gene_symbol": "GNAT2",
  "gene_name": "Guanine nucleotide-binding protein G(t) subunit alpha-2",
  "term_id": "GO:0005737",
  "gene": "UniProtKB:P19087"
}